laminin-9 complex [GO:0043258] (cellular component) References: PMID:10842354 Sources: GOC:jl Also known as: laminin-421 complex Relationships: is a type of laminin complex [GO:0043256] Definition: A laminin complex composed of alpha4, beta2 and gamma1 polypeptide chains.